{
  "term_label": "nucleus",
  "gene_symbol": "CDIP1",
  "gene": "UniProtKB:Q9H305",
  "term_id": "GO:0005634",
  "gene_name": "Cell death-inducing p53-target protein 1"
}